beta-alanine catabolic process to L-alanine [GO:0019485] (biological process) Definition: The chemical reactions and pathways resulting in the breakdown of beta-alanine into other compounds, including L-alanine. Also known as: beta-alanine breakdown to L-alanine, beta-alanine degradation to L-alanine Relationships: is a type of GO:0019484; is a type of L-alanine metabolic process [GO:0042851] Sources: GOC:go_curators